symbiont-mediated suppression of host-directed shutoff of host translation [GO:0141154] (biological process) Relationships: is a type of GO:0044414 Definition: A process in which a symbiont inhibits or disrupts the host shutoff of host translation, a host response that prevents mRNA in the cell to be translated, to prevent the symbiont from expressing its genes. The host is defined as the larger of the organisms involved in a symbiotic interaction. Subtypes: symbiont-mediated suppression of host PKR/eIFalpha signaling [GO:0039580] References: PMID:20563710, PMID:21622569